positive regulation of lovastatin biosynthetic process [GO:0140736] (biological process) Definition: Any process that increases the rate, frequency or extent of the chemical reactions and pathways resulting in the formation of lovastin. References: PMID:10334994, PMID:19781329 Also known as: positive regulation of mevacor biosynthetic process, positive regulation of mevinolin biosynthetic process, positive regulation of monacolin K biosynthetic process Relationships: is a type of positive regulation of lipid biosynthetic process [GO:0046889]; is a type of GO:1900734; positively regulates lovastatin biosynthetic process [GO:0140735]